{
  "gene_symbol": "CYP4A11",
  "term_label": "arachidonate monooxygenase activity",
  "gene_name": "Cytochrome P450 4A11",
  "gene": "UniProtKB:Q02928",
  "term_id": "GO:0008391"
}